{
  "term_label": "DNA-binding transcription factor activity, RNA polymerase II-specific",
  "gene_name": "Zinc finger protein 837",
  "term_id": "GO:0000981",
  "gene": "UniProtKB:Q96EG3",
  "gene_symbol": "ZNF837"
}